{
  "term_id": "GO:0031410",
  "gene": "UniProtKB:Q2M3T9",
  "term_label": "cytoplasmic vesicle",
  "gene_symbol": "HYAL4",
  "gene_name": "Hyaluronidase-4"
}